norepinephrine-epinephrine vasoconstriction involved in regulation of systemic arterial blood pressure [GO:0001994] (biological process) Sources: GOC:mtg_cardio, ISBN:0721643949 Also known as: noradrenaline-adrenaline vasoconstriction involved in regulation of blood pressure, norepinephrine-epinephrine vasoconstriction during blood pressure regulation, norepinephrine-epinephrine vasoconstriction during blood pressure control, norepinephrine-epinephrine vasoconstriction during control of blood pressure Definition: A process that results in a decrease in the diameter of an artery during the norepinephrine-epinephrine response to decreased blood pressure. Relationships: is a type of GO:0042310; is part of positive regulation of blood pressure by epinephrine-norepinephrine [GO:0003321]